{
  "term_id": "GO:0005737",
  "gene_symbol": "NPPA",
  "term_label": "cytoplasm",
  "gene": "UniProtKB:P01160",
  "gene_name": "Natriuretic peptides A"
}